transketolase activity [GO:0004802] (molecular function) Also known as: fructose 6-phosphate:D-glyceraldehyde-3-phosphate glycolaldehydetransferase activity, sedoheptulose-7-phosphate:D-glyceraldehyde-3-phosphate glycolaldehydetransferase activity, glycoaldehyde transferase activity, glycolaldehydetransferase activity Definition: Catalysis of the reversible transfer of a 2-carbon ketol group (CH2OH-CO-) from a ketose phosphate donor to an aldose phosphate acceptor. Relationships: is a type of transketolase or transaldolase activity [GO:0016744] Sources: EC:2.2.1.1, GOC:fmc